{
  "gene_symbol": "GNAZ",
  "term_id": "GO:0031683",
  "term_label": "G-protein beta/gamma-subunit complex binding",
  "gene_name": "Guanine nucleotide-binding protein G(z) subunit alpha",
  "gene": "UniProtKB:P19086"
}